{
  "term_label": "olfactory receptor activity",
  "gene_name": "Olfactory receptor 6C75",
  "gene": "UniProtKB:A6NL08",
  "term_id": "GO:0004984",
  "gene_symbol": "OR6C75"
}